{
  "gene_name": "Nuclear factor interleukin-3-regulated protein",
  "gene_symbol": "NFIL3",
  "gene": "UniProtKB:Q16649",
  "term_label": "regulation of DNA-templated transcription",
  "term_id": "GO:0006355"
}